{
  "gene_symbol": "POLE",
  "term_label": "leading strand elongation",
  "gene_name": "DNA polymerase epsilon catalytic subunit A",
  "gene": "UniProtKB:Q07864",
  "term_id": "GO:0006272"
}